{
  "gene": "UniProtKB:Q9P2N2",
  "term_label": "cytoplasm",
  "gene_symbol": "ARHGAP28",
  "gene_name": "Rho GTPase-activating protein 28",
  "term_id": "GO:0005737"
}